{
  "gene": "UniProtKB:O60896",
  "gene_name": "Receptor activity-modifying protein 3",
  "gene_symbol": "RAMP3",
  "term_id": "GO:0007186",
  "term_label": "G protein-coupled receptor signaling pathway"
}